regulation of nucleus organization [GO:1903353] (biological process) Relationships: is a type of regulation of organelle organization [GO:0033043]; regulates GO:0006997 Definition: Any process that modulates the frequency, rate or extent of nucleus organization. Also known as: regulation of nuclear organisation, regulation of nuclear organization, regulation of nuclear morphology, regulation of nuclear organization and biogenesis, regulation of nucleus organization and biogenesis References: PMID:16943282 Sources: GOC:TermGenie, GO_REF:0000058 Subtypes: regulation of karyogamy [GO:0032871], GO:0045700